retinal cell programmed cell death [GO:0046666] (biological process) Definition: Programmed cell death that occurs in the developing retina. Sources: GOC:bf Also known as: programmed cell death, retina cells, programmed cell death, retinal cells, retina cell programmed cell death, retina programmed cell death, retinal programmed cell death Relationships: is a type of programmed cell death involved in cell development [GO:0010623]; is part of eye morphogenesis [GO:0048592] Subtypes: compound eye retinal cell programmed cell death [GO:0046667] Regulation: regulated by regulation of retinal cell programmed cell death [GO:0046668]; RO_0002213 by positive regulation of retinal cell programmed cell death [GO:0046670]; negatively regulated by negative regulation of retinal cell programmed cell death [GO:0046671]